protein localization to cell leading edge [GO:1902463] (biological process) Relationships: is_a intracellular protein localization [GO:0008104] Definition: A process in which a protein is transported to, or maintained in, a location within a cell leading edge. Also known as: protein localisation in cell leading edge, protein localisation to cell leading edge, protein localization in cell leading edge References: PMID:21543326 Sources: GOC:TermGenie, GOC:lb Regulation: regulated by GO:1905871; RO_0002212 by GO:1905872; positively regulated by positive regulation of protein localization to cell leading edge [GO:1905873]